{
  "term_label": "animal organ development",
  "gene_symbol": "FXR1",
  "gene_name": "RNA-binding protein FXR1",
  "term_id": "GO:0048513",
  "gene": "UniProtKB:P51114"
}